{
  "gene_name": "C-C motif chemokine 4",
  "gene": "UniProtKB:P13236",
  "gene_symbol": "CCL4",
  "term_label": "antimicrobial humoral immune response mediated by antimicrobial peptide",
  "term_id": "GO:0061844"
}